{
  "term_id": "GO:0005886",
  "gene_symbol": "IL1RAP",
  "term_label": "plasma membrane",
  "gene": "UniProtKB:Q9NPH3",
  "gene_name": "Interleukin-1 receptor accessory protein"
}